{
  "gene_symbol": "SLC26A4",
  "term_label": "chloride transmembrane transport",
  "gene_name": "Pendrin",
  "term_id": "GO:1902476",
  "gene": "UniProtKB:O43511"
}